{
  "gene_symbol": "EFTUD2",
  "term_id": "GO:0046540",
  "gene": "UniProtKB:Q15029",
  "term_label": "U4/U6 x U5 tri-snRNP complex",
  "gene_name": "116 kDa U5 small nuclear ribonucleoprotein component"
}